acrosomal matrix [GO:0043159] (cellular component) Relationships: is a type of GO:0110165; is part of acrosomal vesicle [GO:0001669]; is part of vacuole [GO:0005773] References: PMID:8949900, PMID:9139729 Sources: GOC:jl Definition: A structural framework, or 'dense core' at the interior of an acrosome. May regulate the distribution of hydrolases within the acrosome and their release during the acrosome reaction.